{
  "gene": "UniProtKB:P50395",
  "gene_name": "Rab GDP dissociation inhibitor beta",
  "gene_symbol": "GDI2",
  "term_id": "GO:0005829",
  "term_label": "cytosol"
}